{
  "gene_symbol": "CFAP97D1",
  "term_label": "sperm axoneme assembly",
  "gene": "UniProtKB:B2RV13",
  "term_id": "GO:0007288",
  "gene_name": "Sperm axonemal maintenance protein CFAP97D1"
}